{
  "term_label": "cell adhesion",
  "gene": "UniProtKB:Q9Y5E4",
  "term_id": "GO:0007155",
  "gene_symbol": "PCDHB5",
  "gene_name": "Protocadherin beta-5"
}